{
  "gene": "UniProtKB:P68400",
  "gene_name": "Casein kinase II subunit alpha",
  "term_id": "GO:0006302",
  "gene_symbol": "CSNK2A1",
  "term_label": "double-strand break repair"
}